{
  "gene_symbol": "MEGF6",
  "term_id": "GO:0005044",
  "term_label": "scavenger receptor activity",
  "gene": "UniProtKB:O75095",
  "gene_name": "Multiple epidermal growth factor-like domains protein 6"
}